{
  "term_label": "nucleotide-excision repair complex",
  "term_id": "GO:0000109",
  "gene_name": "DNA excision repair protein ERCC-8",
  "gene_symbol": "ERCC8",
  "gene": "UniProtKB:Q13216"
}